{
  "term_id": "UNKNOWN:0003",
  "gene_symbol": "LCE3B",
  "term_label": "Unknown cellular component",
  "gene": "UniProtKB:Q5TA77",
  "gene_name": "Late cornified envelope protein 3B"
}